{
  "gene": "UniProtKB:P48448",
  "gene_symbol": "ALDH3B2",
  "gene_name": "Aldehyde dehydrogenase family 3 member B2",
  "term_label": "aldehyde metabolic process",
  "term_id": "GO:0006081"
}